{
  "gene": "UniProtKB:Q16891",
  "gene_symbol": "IMMT",
  "term_label": "MICOS complex",
  "term_id": "GO:0061617",
  "gene_name": "MICOS complex subunit MIC60"
}